{
  "term_id": "GO:0010468",
  "term_label": "regulation of gene expression",
  "gene_name": "Caveolae-associated protein 4",
  "gene": "UniProtKB:Q5BKX8",
  "gene_symbol": "CAVIN4"
}